{
  "gene": "UniProtKB:Q9UQ26",
  "gene_name": "Regulating synaptic membrane exocytosis protein 2",
  "term_id": "GO:0098831",
  "gene_symbol": "RIMS2",
  "term_label": "presynaptic active zone cytoplasmic component"
}